{
  "term_id": "GO:0003678",
  "gene_name": "Regulator of telomere elongation helicase 1",
  "term_label": "DNA helicase activity",
  "gene_symbol": "RTEL1",
  "gene": "UniProtKB:Q9NZ71"
}